{
  "gene_name": "1-acyl-sn-glycerol-3-phosphate acyltransferase epsilon",
  "term_label": "acyltransferase activity",
  "gene": "UniProtKB:Q9NUQ2",
  "gene_symbol": "AGPAT5",
  "term_id": "GO:0016746"
}